{
  "term_id": "GO:0005634",
  "gene_name": "Intestine-specific homeobox",
  "gene": "UniProtKB:Q2M1V0",
  "term_label": "nucleus",
  "gene_symbol": "ISX"
}